prephenate dehydrogenase (NAD+) activity [GO:0008977] (molecular function) Sources: EC:1.3.1.12, RHEA:13869 Relationships: is a type of oxidoreductase activity, acting on the CH-CH group of donors, NAD or NADP as acceptor [GO:0016628] Also known as: hydroxyphenylpyruvate synthase activity, chorismate mutase--prephenate dehydrogenase activity, prephenate:NAD+ oxidoreductase (decarboxylating) Definition: Catalysis of the reaction: NAD+ + prephenate = (4-hydroxyphenyl)pyruvate + CO2 + NADH.